{
  "term_label": "plasma membrane",
  "gene_symbol": "DRD1",
  "gene": "UniProtKB:P21728",
  "term_id": "GO:0005886",
  "gene_name": "D(1A) dopamine receptor"
}